{
  "term_id": "GO:0000226",
  "gene": "UniProtKB:Q9BQE3",
  "term_label": "microtubule cytoskeleton organization",
  "gene_symbol": "TUBA1C",
  "gene_name": "Tubulin alpha-1C chain"
}